{
  "gene_symbol": "CDH8",
  "term_id": "GO:0045296",
  "term_label": "cadherin binding",
  "gene": "UniProtKB:P55286",
  "gene_name": "Cadherin-8"
}